{
  "term_label": "regulation of hippo signaling",
  "gene": "UniProtKB:Q9ULE0",
  "gene_symbol": "WWC3",
  "term_id": "GO:0035330",
  "gene_name": "Protein WWC3"
}